{
  "gene": "UniProtKB:A6NMX2",
  "term_id": "GO:0000340",
  "gene_name": "Eukaryotic translation initiation factor 4E type 1B",
  "gene_symbol": "EIF4E1B",
  "term_label": "RNA 7-methylguanosine cap binding"
}